{
  "term_id": "UNKNOWN:0001",
  "gene": "UniProtKB:Q6UY14",
  "gene_name": "ADAMTS-like protein 4",
  "term_label": "Unknown molecular function",
  "gene_symbol": "ADAMTSL4"
}